{
  "term_label": "intracellular protein transport",
  "gene_name": "ADP-ribosylation factor-like protein 17",
  "gene": "UniProtKB:Q8IVW1",
  "term_id": "GO:0006886",
  "gene_symbol": "ARL17A"
}